negative regulation of hypoxia-induced intrinsic apoptotic signaling pathway [GO:1903298] (biological process) References: PMID:24553947 Sources: GOC:PARL, GOC:TermGenie, GOC:bf, GO_REF:0000058 Relationships: is a type of GO:1900038; is a type of regulation of hypoxia-induced intrinsic apoptotic signaling pathway [GO:1903297]; is a type of negative regulation of intrinsic apoptotic signaling pathway [GO:2001243]; negatively regulates intrinsic apoptotic signaling pathway in response to hypoxia [GO:1990144] Definition: Any process that stops, prevents or reduces the frequency, rate or extent of hypoxia-induced intrinsic apoptotic signaling pathway. Also known as: down regulation of intrinsic apoptotic signaling pathway in response to hypoxia, down-regulation of intrinsic apoptotic signaling pathway in response to hypoxia, downregulation of intrinsic apoptotic signaling pathway in response to hypoxia, negative regulation of hypoxic stress-induced intrinsic apoptotic signaling pathway, negative regulation of intrinsic apoptotic signaling pathway in response to hypoxia, inhibition of intrinsic apoptotic signaling pathway in response to hypoxia, negative regulation of hypoxia-induced apoptosis, protection against hypoxia-induced apoptosis